{
  "gene": "UniProtKB:O60664",
  "term_label": "positive regulation of triglyceride storage",
  "gene_name": "Perilipin-3",
  "term_id": "GO:0010890",
  "gene_symbol": "PLIN3"
}